negative regulation of mast cell cytokine production [GO:0032764] (biological process) Also known as: down regulation of mast cell cytokine production, down-regulation of mast cell cytokine production, downregulation of mast cell cytokine production, inhibition of mast cell cytokine production Definition: Any process that stops, prevents, or reduces the frequency, rate, or extent of mast cell cytokine production. Sources: GOC:mah Relationships: is a type of negative regulation of cytokine production involved in immune response [GO:0002719]; is a type of regulation of mast cell cytokine production [GO:0032763]; negatively regulates mast cell cytokine production [GO:0032762]